{
  "term_id": "UNKNOWN:0001",
  "term_label": "Unknown molecular function",
  "gene": "UniProtKB:Q2VPA4",
  "gene_name": "Complement component receptor 1-like protein",
  "gene_symbol": "CR1L"
}